{
  "gene": "UniProtKB:Q8TCP9",
  "term_id": "UNKNOWN:0003",
  "gene_symbol": "FAM200A",
  "term_label": "Unknown cellular component",
  "gene_name": "Protein FAM200A"
}